{
  "term_id": "GO:0048666",
  "gene_symbol": "RHOXF2",
  "term_label": "neuron development",
  "gene": "UniProtKB:Q9BQY4",
  "gene_name": "Rhox homeobox family member 2"
}